{
  "term_label": "Unknown biological process",
  "gene": "UniProtKB:Q14507",
  "gene_symbol": "EDDM3A",
  "term_id": "UNKNOWN:0002",
  "gene_name": "Epididymal secretory protein E3-alpha"
}